catechol-containing siderophore biosynthetic process [GO:0019540] (biological process) References: PMID:20376388 Relationships: is a type of catechol-containing compound biosynthetic process [GO:0009713]; is a type of siderophore biosynthetic process [GO:0019290] Definition: The chemical reactions and pathways resulting in the formation of a siderophore from other compounds, including catechol. Catechol is one of the three major chemical groups incorporated into siderophore structures with hydroxamate and a-hydroxycarboxylate, each having a high selectivity for iron(3+). Subtypes: enterobactin biosynthetic process [GO:0009239]